lithium ion binding [GO:0031403] (MF) Relationships: is a type of alkali metal ion binding [GO:0031420] Sources: GOC:mah Definition: Binding to a lithium ion (Li+). Also known as: Li+ ion binding